{
  "term_label": "N-acetylglucosamine metabolic process",
  "gene_symbol": "CHST7",
  "gene_name": "Carbohydrate sulfotransferase 7",
  "gene": "UniProtKB:Q9NS84",
  "term_id": "GO:0006044"
}